{
  "term_label": "Unknown biological process",
  "gene_symbol": "MINPP1",
  "term_id": "UNKNOWN:0002",
  "gene_name": "Multiple inositol polyphosphate phosphatase 1",
  "gene": "UniProtKB:Q9UNW1"
}